{
  "gene_symbol": "RNF19B",
  "gene_name": "E3 ubiquitin-protein ligase RNF19B",
  "gene": "UniProtKB:Q6ZMZ0",
  "term_id": "GO:0031624",
  "term_label": "ubiquitin conjugating enzyme binding"
}